{
  "term_label": "Unknown cellular component",
  "term_id": "UNKNOWN:0003",
  "gene": "UniProtKB:O43299",
  "gene_name": "AP-5 complex subunit zeta-1",
  "gene_symbol": "AP5Z1"
}